{
  "gene_symbol": "ZBTB42",
  "term_label": "DNA-binding transcription factor activity, RNA polymerase II-specific",
  "term_id": "GO:0000981",
  "gene": "UniProtKB:B2RXF5",
  "gene_name": "Zinc finger and BTB domain-containing protein 42"
}